actomyosin contractile ring [GO:0005826] (cellular component) Also known as: CAR, contractile actomyosin ring, actomyosin ring, constriction ring, cytokinetic ring Relationships: is a type of contractile ring [GO:0070938]; is part of cortical actin cytoskeleton [GO:0030864]; is part of cell division site [GO:0032153] Definition: A cytoskeletal structure composed of actin filaments and myosin that forms beneath the plasma membrane of many cells, including animal cells and yeast cells, in a plane perpendicular to the axis of the spindle, i.e. the cell division plane. In animal cells, the contractile ring is located at the cleavage furrow. In budding fungal cells, e.g. mitotic S. cerevisiae cells, the contractile ring forms at the mother-bud neck before mitosis. Subtypes: mitotic actomyosin contractile ring [GO:0110085], GO:0110086 References: PMID:28914606 Sources: GOC:expert_jrp, GOC:sgd_curators, GOC:vw, ISBN:0805319409, ISBN:0815316194